{
  "gene_name": "Putative fatty acid-binding protein 5-like protein 3",
  "term_label": "fatty acid transport",
  "gene_symbol": "FABP5P3",
  "gene": "UniProtKB:A8MUU1",
  "term_id": "GO:0015908"
}